{
  "term_label": "cytoplasmic side of plasma membrane",
  "gene_symbol": "SAMD12",
  "gene": "UniProtKB:Q8N8I0",
  "gene_name": "Sterile alpha motif domain-containing protein 12",
  "term_id": "GO:0009898"
}